{
  "gene_symbol": "TMEM184C",
  "term_id": "GO:0022857",
  "gene": "UniProtKB:Q9NVA4",
  "term_label": "transmembrane transporter activity",
  "gene_name": "Transmembrane protein 184C"
}